{
  "gene": "UniProtKB:Q9NQC7",
  "gene_symbol": "CYLD",
  "gene_name": "Ubiquitin carboxyl-terminal hydrolase CYLD",
  "term_label": "regulation of intrinsic apoptotic signaling pathway",
  "term_id": "GO:2001242"
}